{
  "gene": "UniProtKB:Q9NY57",
  "gene_symbol": "STK32B",
  "term_label": "Unknown cellular component",
  "gene_name": "Serine_threonine-protein kinase 32B",
  "term_id": "UNKNOWN:0003"
}